{
  "gene_name": "Cytochrome P450 4A11",
  "gene_symbol": "CYP4A11",
  "gene": "UniProtKB:Q02928",
  "term_label": "kidney development",
  "term_id": "GO:0001822"
}